{
  "gene_name": "HIV Tat-specific factor 1",
  "gene_symbol": "HTATSF1",
  "gene": "UniProtKB:O43719",
  "term_label": "U2 snRNP",
  "term_id": "GO:0005686"
}